{
  "term_label": "chromatin",
  "gene_name": "MAX gene-associated protein",
  "gene": "UniProtKB:Q8IWI9",
  "term_id": "GO:0000785",
  "gene_symbol": "MGA"
}